{
  "gene_name": "Olfactory receptor 8K5",
  "gene_symbol": "OR8K5",
  "term_id": "UNKNOWN:0001",
  "gene": "UniProtKB:Q8NH50",
  "term_label": "Unknown molecular function"
}